{
  "gene_name": "Microphthalmia-associated transcription factor",
  "term_label": "DNA-binding transcription factor activity, RNA polymerase II-specific",
  "gene_symbol": "MITF",
  "term_id": "GO:0000981",
  "gene": "UniProtKB:O75030"
}